{
  "gene": "UniProtKB:Q9BZC1",
  "term_label": "mRNA binding",
  "gene_symbol": "CELF4",
  "gene_name": "CUGBP Elav-like family member 4",
  "term_id": "GO:0003729"
}